{
  "gene": "UniProtKB:P0C7T2",
  "term_id": "GO:0004984",
  "gene_symbol": "OR2T7",
  "term_label": "olfactory receptor activity",
  "gene_name": "Olfactory receptor 2T7"
}